{
  "gene_symbol": "GLYCAM1",
  "gene_name": "Putative glycosylation-dependent cell adhesion molecule 1",
  "gene": "UniProtKB:Q8IVK1",
  "term_id": "UNKNOWN:0002",
  "term_label": "Unknown biological process"
}